lincomycin catabolic process [GO:1901773] (biological process) Also known as: lincomycin breakdown, lincomycin catabolism, lincomycin degradation Relationships: is a type of S-glycoside catabolic process [GO:0016145]; is a type of modified amino acid catabolic process [GO:0042219]; is a type of amide metabolic process [GO:0043603] Definition: The chemical reactions and pathways resulting in the breakdown of lincomycin. References: PMID:8577249 Sources: GOC:TermGenie, GOC:yaf